ceramide floppase activity [GO:0099038] (MF) Also known as: ATP-dependent ceramide transporter activity, ATPase-coupled ceramide transporter activity, ceramide-translocating ATPase activity, ceramide floppase activity (cytosolic to exoplasmic leaflet) Sources: GOC:BHF, GOC:dos, GOC:rl Definition: Catalysis of the movement of ceramide from the cytosolic to the exoplasmic leaflet of a membrane, using energy from the hydrolysis of ATP. Relationships: is_a sphingolipid floppase activity [GO:0046623]; is part of ceramide translocation [GO:0099040]